{
  "term_label": "RNA polymerase II cis-regulatory region sequence-specific DNA binding",
  "gene": "UniProtKB:Q92753",
  "gene_symbol": "RORB",
  "term_id": "GO:0000978",
  "gene_name": "Nuclear receptor ROR-beta"
}